peptidoglycan stem peptide endopeptidase activity [GO:0061786] (MF) Relationships: is a type of peptidoglycan endopeptidase activity [GO:0061785] References: PMID:22748813 Sources: GOC:dph, GOC:jh Definition: A peptidoglycan endopeptidase activity that acts on a stem peptide of peptidoglycan.